{
  "term_label": "ferrous iron transmembrane transporter activity",
  "gene_name": "Natural resistance-associated macrophage protein 2",
  "gene_symbol": "SLC11A2",
  "gene": "UniProtKB:P49281",
  "term_id": "GO:0015093"
}